 [go#goslim:prokaryote:ribbon] Note: Prokaryote GO ribbon slim